{
  "term_label": "nucleus",
  "term_id": "GO:0005634",
  "gene_name": "Zinc finger protein 879",
  "gene_symbol": "ZNF879",
  "gene": "UniProtKB:B4DU55"
}